{
  "term_id": "UNKNOWN:0001",
  "gene": "UniProtKB:Q8N6M5",
  "gene_name": "Probable inactive allantoicase",
  "gene_symbol": "ALLC",
  "term_label": "Unknown molecular function"
}